{
  "term_label": "adenylate cyclase-activating G protein-coupled receptor signaling pathway",
  "term_id": "GO:0007189",
  "gene": "UniProtKB:Q92633",
  "gene_name": "Lysophosphatidic acid receptor 1",
  "gene_symbol": "LPAR1"
}